{
  "term_id": "GO:0009378",
  "term_label": "four-way junction helicase activity",
  "gene": "UniProtKB:Q14191",
  "gene_name": "Bifunctional 3'-5' exonuclease_ATP-dependent helicase WRN",
  "gene_symbol": "WRN"
}